{
  "gene_name": "Aspartyl_asparaginyl beta-hydroxylase",
  "term_id": "GO:0062101",
  "gene": "UniProtKB:Q12797",
  "gene_symbol": "ASPH",
  "term_label": "peptidyl-aspartic acid 3-dioxygenase activity"
}